{
  "term_label": "negative regulation of DNA-templated transcription",
  "term_id": "GO:0045892",
  "gene": "UniProtKB:Q7L4P6",
  "gene_symbol": "BEND5",
  "gene_name": "BEN domain-containing protein 5"
}